delta7-sterol 5(6)-desaturase activity [GO:0050046] (molecular function) Definition: Catalysis of the reaction: a Delta(7)-sterol + 2 Fe(II)-[cytochrome b5] + O2 + 2 H+ = a Delta(5),Delta(7)-sterol + 2 Fe(III)-[cytochrome b5] + 2 H2O. Also known as: lathosterol oxidase activity, 5-DES, delta7-sterol 5-desaturase activity, delta7-sterol delta5-dehydrogenase activity, delta7-sterol-C5(6)-desaturase activity, lathosterol 5-desaturase activity Relationships: is a type of GO:0070704 Sources: RHEA:54320